{
  "gene": "UniProtKB:Q9BYV7",
  "term_label": "mitochondrion",
  "gene_symbol": "BCO2",
  "term_id": "GO:0005739",
  "gene_name": "Carotenoid-cleaving dioxygenase, mitochondrial"
}